negative regulation of antigen processing and presentation of polysaccharide antigen via MHC class II [GO:0002602] (biological process) Also known as: down regulation of antigen processing and presentation of polysaccharide antigen via MHC class II, down-regulation of antigen processing and presentation of polysaccharide antigen via MHC class II, downregulation of antigen processing and presentation of polysaccharide antigen via MHC class II, negative regulation of polysaccharide antigen processing and presentation via MHC class II, inhibition of antigen processing and presentation of polysaccharide antigen via MHC class II Sources: GOC:add Definition: Any process that stops, prevents, or reduces the frequency, rate, or extent of antigen processing and presentation of polysaccharide antigen via MHC class II. Relationships: is a type of GO:0002581; is a type of regulation of antigen processing and presentation of polysaccharide antigen via MHC class II [GO:0002601]; negatively regulates antigen processing and presentation of polysaccharide antigen via MHC class II [GO:0002505]